{
  "gene_symbol": "TCF21",
  "term_id": "GO:0032502",
  "term_label": "developmental process",
  "gene": "UniProtKB:O43680",
  "gene_name": "Transcription factor 21"
}